{
  "term_id": "GO:0097116",
  "term_label": "gephyrin clustering involved in postsynaptic density assembly",
  "gene_symbol": "NRXN1",
  "gene": "UniProtKB:Q9ULB1",
  "gene_name": "Neurexin-1"
}